response to gemcitabine [GO:0036272] (biological process) Relationships: is a type of response to nitrogen compound [GO:1901698]; is a type of GO:1901700 Note: Note that this term is in the subset of terms that should not be used for direct manual annotation of gene products. It was created to be used for cross-referencing by other ontologies. Direct annotations to this term may be amended during annotation QC. Sources: GOC:hp, Wikipedia:Gemcitabine Also known as: response to 2',2'-difluorodeoxycytidine, response to 2'-deoxy-2',2'-difluorocytidine Definition: Any process that results in a change in state or activity of a cell or an organism (in terms of movement, secretion, enzyme production, gene expression, etc.) as a result of a gemcitabine stimulus. Gemcitabine is a 2'-deoxycytidine having geminal fluoro substituents in the 2'-position, and is used as a drug in the treatment of various carcinomas.